{
  "term_id": "UNKNOWN:0003",
  "gene_symbol": "LIMS3",
  "gene": "UniProtKB:P0CW19",
  "gene_name": "LIM and senescent cell antigen-like-containing domain protein 3",
  "term_label": "Unknown cellular component"
}